{
  "gene_symbol": "PDIA4",
  "term_label": "cell surface",
  "term_id": "GO:0009986",
  "gene_name": "Protein disulfide-isomerase A4",
  "gene": "UniProtKB:P13667"
}